{
  "gene": "UniProtKB:Q8IXT5",
  "term_id": "GO:0003723",
  "term_label": "RNA binding",
  "gene_name": "RNA-binding protein 12B",
  "gene_symbol": "RBM12B"
}